negative regulation of prostatic bud formation [GO:0060686] (biological process) Definition: Any process that decreases the rate, frequency, or extent of prostatic bud formation, the morphogenetic process in which a region of the fetal urogenital sinus epithelium is specified to become the prostate, resulting in prostate bud outgrowth. Sources: GOC:dph Relationships: is a type of GO:0060685; is a type of negative regulation of morphogenesis of an epithelium [GO:1905331]; is a type of negative regulation of reproductive process [GO:2000242]; negatively regulates prostatic bud formation [GO:0060513]